{
  "gene": "UniProtKB:P0CW20",
  "term_label": "Unknown biological process",
  "gene_symbol": "LIMS4",
  "gene_name": "LIM and senescent cell antigen-like-containing domain protein 4",
  "term_id": "UNKNOWN:0002"
}